{
  "term_label": "cellular response to interferon-beta",
  "gene_name": "Pyrin and HIN domain-containing protein 1",
  "gene": "UniProtKB:Q6K0P9",
  "gene_symbol": "PYHIN1",
  "term_id": "GO:0035458"
}